{
  "gene": "UniProtKB:P10276",
  "gene_name": "Retinoic acid receptor alpha",
  "term_id": "GO:0030154",
  "gene_symbol": "RARA",
  "term_label": "cell differentiation"
}